paraxial mesodermal cell fate commitment [GO:0048343] (biological process) Relationships: is a type of mesodermal cell fate commitment [GO:0001710]; is part of paraxial mesodermal cell differentiation [GO:0048342] Definition: The process in which a cell becomes committed to become a paraxial mesoderm cell. Sources: GOC:dgh